{
  "gene_symbol": "PPP1R1C",
  "term_id": "UNKNOWN:0001",
  "term_label": "Unknown molecular function",
  "gene_name": "Protein phosphatase 1 regulatory subunit 1C",
  "gene": "UniProtKB:Q8WVI7"
}